{
  "gene_symbol": "OR10S1",
  "gene_name": "Olfactory receptor 10S1",
  "gene": "UniProtKB:Q8NGN2",
  "term_id": "GO:0050911",
  "term_label": "detection of chemical stimulus involved in sensory perception of smell"
}